{
  "gene_symbol": "ESPL1",
  "term_label": "meiotic chromosome separation",
  "gene": "UniProtKB:Q14674",
  "term_id": "GO:0051307",
  "gene_name": "Separin"
}